{
  "gene_symbol": "SMIM32",
  "term_id": "UNKNOWN:0002",
  "term_label": "Unknown biological process",
  "gene": "UniProtKB:A0A1B0GUA5",
  "gene_name": "Small integral membrane protein 32"
}